{
  "gene_symbol": "NHERF1",
  "term_id": "GO:0043495",
  "term_label": "protein-membrane adaptor activity",
  "gene": "UniProtKB:O14745",
  "gene_name": "Na(+)_H(+) exchange regulatory cofactor NHE-RF1"
}